{
  "term_label": "septin complex",
  "gene": "UniProtKB:Q9NVA2",
  "term_id": "GO:0031105",
  "gene_symbol": "SEPTIN11",
  "gene_name": "Septin-11"
}